positive regulation of L-leucine import across plasma membrane [GO:1905534] (biological process) Also known as: positive regulation of leucine import across plasma membrane, positive regulation of L-leucine import into cell, up regulation of L-leucine import into cell, upregulation of L-leucine import into cell, activation of L-leucine import into cell, activation of leucine import into cell References: PMID:10467003 Sources: GOC:TermGenie, GO_REF:0000058 Definition: Any process that activates or increases the frequency, rate or extent of L-leucine import across plasma membrane. Relationships: is a type of positive regulation of organic acid transport [GO:0032892]; is a type of positive regulation of transmembrane transport [GO:0034764]; is a type of positive regulation of amino acid transport [GO:0051957]; is_a regulation of L-leucine import across plasma membrane [GO:1905532]; positively regulates L-leucine import across plasma membrane [GO:1903801]